{
  "term_label": "positive regulation of angiogenesis",
  "gene": "UniProtKB:O95398",
  "gene_symbol": "RAPGEF3",
  "term_id": "GO:0045766",
  "gene_name": "Rap guanine nucleotide exchange factor 3"
}